{
  "gene": "UniProtKB:Q6VVX0",
  "term_id": "GO:0006082",
  "gene_name": "Vitamin D 25-hydroxylase",
  "term_label": "organic acid metabolic process",
  "gene_symbol": "CYP2R1"
}